{
  "gene": "UniProtKB:Q9UMX5",
  "gene_name": "Neudesin",
  "term_id": "GO:0016020",
  "term_label": "membrane",
  "gene_symbol": "NENF"
}